{
  "gene_symbol": "TAFAZZIN",
  "gene": "UniProtKB:Q16635",
  "term_id": "GO:0007007",
  "gene_name": "Tafazzin",
  "term_label": "inner mitochondrial membrane organization"
}